{
  "term_label": "Unknown cellular component",
  "gene_symbol": "OR5W2",
  "gene_name": "Olfactory receptor 5W2",
  "term_id": "UNKNOWN:0003",
  "gene": "UniProtKB:Q8NH69"
}